{
  "term_id": "UNKNOWN:0001",
  "term_label": "Unknown molecular function",
  "gene_symbol": "KCTD3",
  "gene": "UniProtKB:Q9Y597",
  "gene_name": "BTB_POZ domain-containing protein KCTD3"
}